{
  "gene_name": "High affinity immunoglobulin epsilon receptor subunit gamma",
  "gene_symbol": "FCER1G",
  "term_label": "IgE receptor activity",
  "term_id": "GO:0019767",
  "gene": "UniProtKB:P30273"
}